CXCR2 chemokine receptor binding [GO:0045238] (molecular function) References: PMID:11910892 Sources: GOC:ceb Also known as: CXCR2 chemokine receptor ligand Relationships: is a type of interleukin-8 receptor binding [GO:0005153] Definition: Binding to a CXCR2 chemokine receptor.